{
  "gene_symbol": "GTF2A1",
  "term_label": "transcription factor TFIIA complex",
  "term_id": "GO:0005672",
  "gene_name": "Transcription initiation factor IIA subunit 1",
  "gene": "UniProtKB:P52655"
}